{
  "gene_name": "Protein arginine methyltransferase NDUFAF7, mitochondrial",
  "gene": "UniProtKB:Q7L592",
  "term_id": "GO:0032981",
  "gene_symbol": "NDUFAF7",
  "term_label": "mitochondrial respiratory chain complex I assembly"
}